{
  "gene_name": "Putative neutrophil cytosol factor 1B",
  "gene_symbol": "NCF1B",
  "term_id": "GO:0043020",
  "gene": "UniProtKB:A6NI72",
  "term_label": "NADPH oxidase complex"
}